{
  "gene_name": "Adenomatous polyposis coli protein 2",
  "term_label": "gamma-catenin binding",
  "gene": "UniProtKB:O95996",
  "term_id": "GO:0045295",
  "gene_symbol": "APC2"
}